{
  "term_id": "GO:0000226",
  "gene_name": "Thioredoxin domain-containing protein 9",
  "gene": "UniProtKB:O14530",
  "gene_symbol": "TXNDC9",
  "term_label": "microtubule cytoskeleton organization"
}